{
  "term_label": "extracellular region",
  "gene": "UniProtKB:Q8N1E2",
  "gene_symbol": "LYG1",
  "gene_name": "Lysozyme g-like protein 1",
  "term_id": "GO:0005576"
}